{
  "gene": "UniProtKB:O43639",
  "term_id": "GO:1902237",
  "term_label": "positive regulation of endoplasmic reticulum stress-induced intrinsic apoptotic signaling pathway",
  "gene_name": "Cytoplasmic protein NCK2",
  "gene_symbol": "NCK2"
}